muscle cell cellular homeostasis [GO:0046716] (biological process) References: PMID:3091429, PMID:7781901 Sources: GOC:mah Relationships: is a type of cellular homeostasis [GO:0019725] Also known as: muscle fiber maintenance, muscle homeostasis Definition: The cellular homeostatic process that preserves a muscle cell in a stable functional or structural state.